{
  "gene_symbol": "ERGIC1",
  "term_label": "Golgi membrane",
  "gene_name": "Endoplasmic reticulum-Golgi intermediate compartment protein 1",
  "term_id": "GO:0000139",
  "gene": "UniProtKB:Q969X5"
}